dichotomous subdivision of terminal units involved in salivary gland branching [GO:0060666] (biological process) Sources: GOC:dph Relationships: is a type of dichotomous subdivision of an epithelial terminal unit [GO:0060600]; is part of GO:0060445 Definition: The process in which a salivary epithelial cord bifurcates at its end.